{
  "gene_symbol": "GRIP1",
  "term_label": "Unknown molecular function",
  "gene": "UniProtKB:Q9Y3R0",
  "gene_name": "Glutamate receptor-interacting protein 1",
  "term_id": "UNKNOWN:0001"
}